{
  "gene_name": "Sodium_potassium-transporting ATPase subunit alpha-4",
  "gene": "UniProtKB:Q13733",
  "term_id": "GO:0005391",
  "gene_symbol": "ATP1A4",
  "term_label": "P-type sodium:potassium-exchanging transporter activity"
}